{
  "gene": "UniProtKB:Q8NI35",
  "term_label": "apical part of cell",
  "gene_symbol": "PATJ",
  "gene_name": "InaD-like protein",
  "term_id": "GO:0045177"
}